{
  "term_label": "cytoplasm",
  "gene_name": "Kelch-like protein 5",
  "gene": "UniProtKB:Q96PQ7",
  "gene_symbol": "KLHL5",
  "term_id": "GO:0005737"
}